regulation of blood coagulation, extrinsic pathway [GO:2000263] (biological process) Sources: GOC:mah Definition: Any process that modulates the frequency, rate or extent of blood coagulation, extrinsic pathway. Relationships: is a type of regulation of blood coagulation [GO:0030193]; is a type of regulation of protein activation cascade [GO:2000257]; regulates blood coagulation, extrinsic pathway [GO:0007598] Subtypes: GO:2000264, positive regulation of blood coagulation, extrinsic pathway [GO:2000265]